phosphoglucomutase activity [GO:0004614] (molecular function) Sources: EC:5.4.2.2 Definition: Catalysis of the reaction: alpha-D-glucose 1-phosphate = alpha-D-glucose 6-phosphate. Subtypes: phosphoglucomutase (glucose-cofactor) activity [GO:0047468] Also known as: alpha-D-glucose 1,6-phosphomutase activity, glucose phosphomutase activity, phosphoglucose mutase activity Relationships: is a type of intramolecular phosphotransferase activity [GO:0016868]